estradiol secretion [GO:0035938] (biological process) Relationships: is a type of GO:0015850; is a type of steroid hormone secretion [GO:0035929] Definition: The regulated release of estradiol into the circulatory system. References: PMID:21632818 Sources: GOC:sl Regulation: regulated by regulation of estradiol secretion [GO:2000864]; RO_0002212 by negative regulation of estradiol secretion [GO:2000865]; positively regulated by positive regulation of estradiol secretion [GO:2000866] Also known as: oestradiol secretion